{
  "gene": "UniProtKB:Q14139",
  "term_id": "GO:0036503",
  "gene_name": "Ubiquitin conjugation factor E4 A",
  "gene_symbol": "UBE4A",
  "term_label": "ERAD pathway"
}